{
  "gene": "UniProtKB:Q02241",
  "term_id": "GO:0007018",
  "gene_name": "Kinesin-like protein KIF23",
  "gene_symbol": "KIF23",
  "term_label": "microtubule-based movement"
}